{
  "gene_symbol": "AQP1",
  "term_id": "GO:0035379",
  "gene_name": "Aquaporin-1",
  "term_label": "carbon dioxide transmembrane transporter activity",
  "gene": "UniProtKB:P29972"
}